{
  "term_id": "GO:0048471",
  "gene_name": "Spermatid-specific manchette-related protein 1",
  "term_label": "perinuclear region of cytoplasm",
  "gene_symbol": "SMRP1",
  "gene": "UniProtKB:Q8NCR6"
}